{
  "gene": "UniProtKB:Q4J6C6",
  "gene_symbol": "PREPL",
  "gene_name": "Prolyl endopeptidase-like",
  "term_label": "Unknown biological process",
  "term_id": "UNKNOWN:0002"
}